positively regulates [RO:0002213] (external) Relationships: subPropertyOf regulates [RO:0002211]